pyrimidine nucleotide catabolic process [GO:0006244] (biological process) Also known as: pyrimidine nucleotide breakdown, pyrimidine nucleotide catabolism, pyrimidine nucleotide degradation Subtypes: pyrimidine ribonucleotide catabolic process [GO:0009222], GO:0009223 Relationships: is a type of pyrimidine nucleotide metabolic process [GO:0006220]; is a type of GO:0009166; is a type of pyrimidine-containing compound catabolic process [GO:0072529] Definition: The chemical reactions and pathways resulting in the breakdown of a pyrimidine nucleotide, a compound consisting of nucleoside (a pyrimidine base linked to a deoxyribose or ribose sugar) esterified with a phosphate group at either the 3' or 5'-hydroxyl group of the sugar. Sources: GOC:go_curators, ISBN:0198506732